{
  "gene_name": "E3 ubiquitin-protein ligase RLIM",
  "term_label": "random inactivation of X chromosome",
  "term_id": "GO:0060816",
  "gene_symbol": "RLIM",
  "gene": "UniProtKB:Q9NVW2"
}